{
  "gene": "UniProtKB:Q9GZR5",
  "term_label": "fatty acid elongation, polyunsaturated fatty acid",
  "gene_symbol": "ELOVL4",
  "term_id": "GO:0034626",
  "gene_name": "Elongation of very long chain fatty acids protein 4"
}